ta-siRNA processing [GO:0010267] (biological process) References: PMID:16129836, PMID:20687832 Sources: GOC:tb Also known as: RNA interference, production of ta-siRNAs, primary ta-siRNA processing, production of ta-siRNAs involved in RNA interference, production of small RNA involved in gene silencing by RNA Definition: A process leading to the generation of a functional trans-acting small interfering RNA (ta-siRNA). ta-siRNAs function like miRNAs to guide cleavage of target mRNAs. Relationships: is a type of siRNA processing [GO:0030422]